{
  "term_id": "UNKNOWN:0001",
  "gene_name": "Melanoma-associated antigen B18",
  "term_label": "Unknown molecular function",
  "gene_symbol": "MAGEB18",
  "gene": "UniProtKB:Q96M61"
}